negative regulation of B cell antigen processing and presentation [GO:0002623] (BP) Definition: Any process that stops, prevents, or reduces the frequency, rate, or extent of B cell antigen processing and presentation. Sources: GOC:add Also known as: down regulation of B cell antigen processing and presentation, down-regulation of B cell antigen processing and presentation, downregulation of B cell antigen processing and presentation, negative regulation of B lymphocyte antigen processing and presentation, negative regulation of B-cell antigen processing and presentation, negative regulation of B-lymphocyte antigen processing and presentation, inhibition of B cell antigen processing and presentation Relationships: is a type of negative regulation of antigen processing and presentation [GO:0002578]; is a type of regulation of B cell antigen processing and presentation [GO:0002622]; is_a negative regulation of B cell mediated immunity [GO:0002713]; negatively regulates GO:0002450